androstan-3-alpha,17-beta-diol dehydrogenase (NAD+) activity [GO:0047044] (molecular function) Relationships: is a type of steroid dehydrogenase activity, acting on the CH-OH group of donors, NAD or NADP as acceptor [GO:0033764] Also known as: 3-alpha(or 20-beta)-hydroxysteroid dehydrogenase activity, 3alpha(or 20beta)-hydroxysteroid dehydrogenase activity, 3alpha(or 20beta)-hydroxysteroid:NAD+ oxidoreductase activity, 3alpha,20beta-hydroxysteroid:NAD+-oxidoreductase activity, NADH-20beta-hydroxysteroid dehydrogenase activity, dehydrogenase, 20beta-hydroxy steroid, delta4-3-ketosteroid hydrogenase activity, (R)-20-hydroxysteroid dehydrogenase activity, 20beta-HSD, 20beta-hydroxysteroid dehydrogenase activity, cortisone reductase activity Definition: Catalysis of the reaction: NAD+ + androstan-3-alpha,17-beta-diol = 17-beta-hydroxyandrostan-3-one + NADH + H+. Sources: RHEA:22400